{
  "term_label": "U1 snRNA 3'-end processing",
  "term_id": "GO:0034473",
  "gene_symbol": "EXOSC7",
  "gene": "UniProtKB:Q15024",
  "gene_name": "Exosome complex component RRP42"
}